{
  "gene": "UniProtKB:Q16572",
  "gene_name": "Vesicular acetylcholine transporter",
  "term_id": "GO:0030122",
  "gene_symbol": "SLC18A3",
  "term_label": "AP-2 adaptor complex"
}